{
  "term_id": "UNKNOWN:0001",
  "gene_symbol": "TMEM50B",
  "gene": "UniProtKB:P56557",
  "gene_name": "Transmembrane protein 50B",
  "term_label": "Unknown molecular function"
}